{
  "gene_name": "Unconventional myosin-Id",
  "term_label": "actin filament organization",
  "term_id": "GO:0007015",
  "gene": "UniProtKB:O94832",
  "gene_symbol": "MYO1D"
}